positive regulation of ovarian follicle development [GO:2000386] (biological process) Relationships: is a type of GO:0051094; is a type of regulation of ovarian follicle development [GO:2000354]; positively regulates GO:0001541 Sources: GOC:obol Also known as: positive regulation of follicular phase Definition: Any process that activates or increases the frequency, rate or extent of ovarian follicle development.